type III interferon-mediated signaling pathway [GO:0038196] (biological process) References: PMID:32464097 Sources: GOC:signaling Relationships: is a type of interferon-mediated signaling pathway [GO:0140888]; is part of GO:0071358 Also known as: type III interferon signaling pathway, type III interferon-activated signaling pathway, interferon lambda signaling pathway Definition: The series of molecular signals initiated by type III interferon binding to its receptor on the surface of a target cell, and ending with the regulation of a downstream cellular process, e.g. transcription. Interferon lambda is the only member of the type III interferon found so far.